{
  "gene": "UniProtKB:Q9Y651",
  "gene_symbol": "SOX21",
  "gene_name": "Transcription factor SOX-21",
  "term_id": "GO:0045944",
  "term_label": "positive regulation of transcription by RNA polymerase II"
}